receptor-receptor interaction [GO:0090722] (molecular function) Definition: The aggregation, arrangement and bonding together of two or more different receptor complexes that individually undergo combination with a hormone, neurotransmitter, drug or intracellular messenger to form a higher level receptor complex. The formation of the higher level complex initiates a change in cell function. Also known as: hetero-receptor complex formation Relationships: is a type of GO:0005102 References: PMID:22035699, PMID:24157794 Sources: GOC:PARL, GOC:dox, GOC:pad